symbiont-mediated perturbation of host programmed cell death [GO:0052040] (biological process) Definition: A process in which a symbiont gene product alters or subverts host programmed cell death, leading to a change in the frequency, rate or extent of host programmed cell death in the host cell. The host is defined as the larger of the organisms involved in a symbiotic interaction. Sources: GOC:curators Also known as: modulation by symbiont of host programmed cell death, modulation of host PCD, modulation by symbiont of host non-apoptotic programmed cell death Relationships: is_a symbiont-mediated perturbation of host cellular process [GO:0044068] Subtypes: symbiont-mediated suppression of host programmed cell death [GO:0052041], symbiont-mediated activation of host programmed cell death [GO:0052042], symbiont-mediated perturbation of host apoptosis [GO:0052150]